{
  "gene": "UniProtKB:P46777",
  "gene_name": "Large ribosomal subunit protein uL18",
  "gene_symbol": "RPL5",
  "term_label": "ribosomal large subunit assembly",
  "term_id": "GO:0000027"
}